{
  "gene_symbol": "KDM6B",
  "term_id": "GO:0010468",
  "term_label": "regulation of gene expression",
  "gene": "UniProtKB:O15054",
  "gene_name": "Lysine-specific demethylase 6B"
}